{
  "gene_name": "LysM and putative peptidoglycan-binding domain-containing protein 1",
  "gene": "UniProtKB:Q96S90",
  "term_label": "Unknown biological process",
  "gene_symbol": "LYSMD1",
  "term_id": "UNKNOWN:0002"
}